{
  "term_id": "UNKNOWN:0002",
  "gene_symbol": "HNRNPR",
  "term_label": "Unknown biological process",
  "gene": "UniProtKB:O43390",
  "gene_name": "Heterogeneous nuclear ribonucleoprotein R"
}